tDNA binding [GO:0071443] (molecular function) Relationships: is a type of sequence-specific double-stranded DNA binding [GO:1990837] Definition: Binding to DNA sequences encoding transfer RNA. Sources: GOC:mah